{
  "term_id": "GO:0004653",
  "gene_symbol": "GALNT14",
  "term_label": "polypeptide N-acetylgalactosaminyltransferase activity",
  "gene": "UniProtKB:Q96FL9",
  "gene_name": "Polypeptide N-acetylgalactosaminyltransferase 14"
}